{
  "gene_symbol": "FSBP",
  "gene_name": "Fibrinogen silencer-binding protein",
  "gene": "UniProtKB:O95073",
  "term_id": "UNKNOWN:0001",
  "term_label": "Unknown molecular function"
}